{
  "term_label": "Unknown molecular function",
  "gene": "UniProtKB:Q5SZL2",
  "gene_symbol": "CEP85L",
  "gene_name": "Centrosomal protein of 85 kDa-like",
  "term_id": "UNKNOWN:0001"
}